{
  "gene": "UniProtKB:Q6UWB4",
  "gene_name": "Serine protease 55",
  "term_id": "GO:0005886",
  "term_label": "plasma membrane",
  "gene_symbol": "PRSS55"
}